chlorosome envelope [GO:0033105] (cellular component) Definition: The structure, composed of a monolayer of glycolipids with embedded proteins, that encloses the pigments and other contents of the chlorosome. References: PMID:14507718, PMID:14729689, PMID:17303128 Relationships: is a type of organelle-enclosing lipid monolayer [GO:0034646]; is part of chlorosome [GO:0046858] Also known as: chlorosome membrane Note: Note that the chlorosome envelope is not a single or double lipid bilayer, so this term is not a child of 'organelle membrane ; GO:0031090' or 'organelle envelope ; GO:0031967'.